{
  "gene_name": "Sperm-associated antigen 5",
  "term_label": "Unknown cellular component",
  "gene": "UniProtKB:Q96R06",
  "term_id": "UNKNOWN:0003",
  "gene_symbol": "SPAG5"
}